{
  "term_label": "cytoplasm",
  "gene": "UniProtKB:Q8N543",
  "term_id": "GO:0005737",
  "gene_symbol": "OGFOD1",
  "gene_name": "Prolyl 3-hydroxylase OGFOD1"
}